{
  "gene_symbol": "SRSF7",
  "term_id": "GO:0000381",
  "gene_name": "Serine_arginine-rich splicing factor 7",
  "gene": "UniProtKB:Q16629",
  "term_label": "regulation of alternative mRNA splicing, via spliceosome"
}